{
  "gene_symbol": "RGS7",
  "gene": "UniProtKB:P49802",
  "term_id": "GO:0005886",
  "term_label": "plasma membrane",
  "gene_name": "Regulator of G-protein signaling 7"
}